{
  "gene": "UniProtKB:Q99714",
  "term_label": "estradiol 17-beta-dehydrogenase [NAD(P)+] activity",
  "gene_name": "3-hydroxyacyl-CoA dehydrogenase type-2",
  "gene_symbol": "HSD17B10",
  "term_id": "GO:0004303"
}